{
  "term_id": "UNKNOWN:0002",
  "gene_name": "RWD domain-containing protein 2B",
  "term_label": "Unknown biological process",
  "gene_symbol": "RWDD2B",
  "gene": "UniProtKB:P57060"
}